{
  "gene_name": "Aldo-keto reductase family 1 member C2",
  "term_label": "androsterone dehydrogenase [NAD(P)+] activity",
  "term_id": "GO:0047023",
  "gene": "UniProtKB:P52895",
  "gene_symbol": "AKR1C2"
}